{
  "gene_symbol": "LSG1",
  "gene_name": "Large subunit GTPase 1 homolog",
  "term_id": "GO:0003924",
  "gene": "UniProtKB:Q9H089",
  "term_label": "GTPase activity"
}